{
  "term_id": "UNKNOWN:0001",
  "term_label": "Unknown molecular function",
  "gene": "UniProtKB:A0A075B6I7",
  "gene_symbol": "IGLV5-48",
  "gene_name": "Probable non-functional immunoglobulin lambda variable 5-48"
}